{
  "term_id": "UNKNOWN:0002",
  "gene_name": "Guanine nucleotide-binding protein-like 1",
  "term_label": "Unknown biological process",
  "gene_symbol": "GNL1",
  "gene": "UniProtKB:P36915"
}